{
  "gene_symbol": "FA2H",
  "gene_name": "Fatty acid 2-hydroxylase",
  "term_id": "GO:0006631",
  "term_label": "fatty acid metabolic process",
  "gene": "UniProtKB:Q7L5A8"
}